{
  "term_label": "ruffle",
  "gene_name": "Inositol polyphosphate 5-phosphatase K",
  "gene": "UniProtKB:Q9BT40",
  "term_id": "GO:0001726",
  "gene_symbol": "INPP5K"
}